sRNA-mediated post-transcriptional gene silencing [GO:0040033] (biological process) Definition: A post-transcriptional gene silencing pathway mediated by the action of small regulatory non-coding RNAs (sRNAs). sRNAs are 20-500 nucleotides in length and found in bacteria. Relationships: is a type of regulatory ncRNA-mediated post-transcriptional gene silencing [GO:0035194] Also known as: RNA-mediated gene silencing by inhibition of translation, downregulation of mRNA translation, ncRNA-mediated, inhibition of mRNA translation, ncRNA-mediated, sRNA-mediated gene silencing, small RNA-mediated gene silencing Note: It is postulated that there 3 mechanisms of sRNA-mediated gene silencing: (i) translation inhibition, (ii) RNA destabilization, and (iii) transcription termination loop formation (as this is common when looking at riboswitches). sRNA mediated gene silencing is sometimes referred to as 'regulation of riboswitch'. References: PMID:12460531, PMID:2468565, PMID:33963446